{
  "gene": "UniProtKB:Q5T2E6",
  "term_id": "GO:0005829",
  "term_label": "cytosol",
  "gene_symbol": "ARMH3",
  "gene_name": "Armadillo-like helical domain-containing protein 3"
}